protein deglycation [GO:0036525] (biological process) Note: Glycation is a non enzymatic covalent addition of a sugar or dicarbonyl (methylglyoxal, glyoxal) to a protein. Deglycation repairs the glycated amino acids. Also known as: glycated protein repair Subtypes: peptidyl-cysteine deglycation [GO:0036526], peptidyl-arginine deglycation [GO:0036527], peptidyl-lysine deglycation [GO:0036528], protein deglycation, glyoxal removal [GO:0036529], protein deglycation, methylglyoxal removal [GO:0036530] References: PMID:14568004, PMID:25416785 Sources: GOC:PARL, GOC:bf Relationships: is_a protein repair [GO:0030091]; is a type of GO:0036211 Definition: The removal of a sugar or dicarbonyl from a glycated protein.